{
  "term_id": "GO:0032281",
  "gene": "UniProtKB:P42262",
  "term_label": "AMPA glutamate receptor complex",
  "gene_name": "Glutamate receptor 2",
  "gene_symbol": "GRIA2"
}